{
  "gene_name": "Secernin-3",
  "term_label": "Unknown molecular function",
  "gene_symbol": "SCRN3",
  "gene": "UniProtKB:Q0VDG4",
  "term_id": "UNKNOWN:0001"
}